{
  "gene_name": "Methanethiol oxidase",
  "gene": "UniProtKB:Q13228",
  "term_label": "Unknown cellular component",
  "term_id": "UNKNOWN:0003",
  "gene_symbol": "SELENBP1"
}